{
  "term_label": "Unknown molecular function",
  "gene": "UniProtKB:A0A075B713",
  "gene_name": "T cell receptor alpha joining 1 (non-functional) (Fragment)",
  "term_id": "UNKNOWN:0001",
  "gene_symbol": "TRAJ1"
}